{
  "gene": "UniProtKB:A8MVW5",
  "term_label": "Unknown molecular function",
  "gene_symbol": "HEPACAM2",
  "term_id": "UNKNOWN:0001",
  "gene_name": "HEPACAM family member 2"
}